{
  "term_id": "GO:0005739",
  "gene_name": "Cytochrome P450 1B1",
  "gene_symbol": "CYP1B1",
  "term_label": "mitochondrion",
  "gene": "UniProtKB:Q16678"
}